{
  "term_label": "defense response to virus",
  "term_id": "GO:0051607",
  "gene_symbol": "IFITM1",
  "gene": "UniProtKB:P13164",
  "gene_name": "Interferon-induced transmembrane protein 1"
}